{
  "term_id": "GO:0005634",
  "gene": "UniProtKB:Q05923",
  "term_label": "nucleus",
  "gene_symbol": "DUSP2",
  "gene_name": "Dual specificity protein phosphatase 2"
}